corrin catabolic process [GO:0046141] (BP) Sources: GOC:ai Relationships: is a type of tetrapyrrole catabolic process [GO:0033015] Definition: The chemical reactions and pathways resulting in the breakdown of corrin, C19H22N4, the fundamental heterocyclic skeleton of the corrinoids. It consists of four reduced pyrrole rings joined into a macrocyclic ring. Corrin is the core of the vitamin B12 molecule. Also known as: corrin breakdown, corrin catabolism, corrin degradation